{
  "gene_name": "Baculoviral IAP repeat-containing protein 7",
  "gene_symbol": "BIRC7",
  "gene": "UniProtKB:Q96CA5",
  "term_label": "negative regulation of apoptotic process",
  "term_id": "GO:0043066"
}